{
  "gene": "UniProtKB:O60383",
  "gene_name": "Growth_differentiation factor 9",
  "term_id": "GO:0005615",
  "gene_symbol": "GDF9",
  "term_label": "extracellular space"
}